positive regulation of glycogen metabolic process [GO:0070875] (biological process) Sources: GOC:mah Relationships: is a type of positive regulation of macromolecule metabolic process [GO:0010604]; is_a positive regulation of glucose metabolic process [GO:0010907]; is a type of GO:0070873; positively regulates GO:0005977 Subtypes: GO:0045725, positive regulation of glycogen catabolic process [GO:0045819] Definition: Any process that activates or increases the frequency, rate or extent of the chemical reactions and pathways involving glycogen. Also known as: positive regulation of glycogen metabolism